{
  "gene_name": "Protein RER1",
  "gene_symbol": "RER1",
  "gene": "UniProtKB:O15258",
  "term_id": "UNKNOWN:0001",
  "term_label": "Unknown molecular function"
}